regulation of sarcinapterin biosynthetic process [GO:1900971] (biological process) Relationships: is a type of regulation of biosynthetic process [GO:0009889]; is a type of regulation of phosphorus metabolic process [GO:0051174]; is a type of regulation of small molecule metabolic process [GO:0062012]; regulates sarcinapterin biosynthetic process [GO:1900868] Subtypes: negative regulation of sarcinapterin biosynthetic process [GO:1900972], positive regulation of sarcinapterin biosynthetic process [GO:1900973] Also known as: regulation of sarcinapterin anabolism, regulation of sarcinapterin biosynthesis, regulation of sarcinapterin formation, regulation of sarcinapterin synthesis Sources: GOC:TermGenie, GOC:mengo_curators Definition: Any process that modulates the frequency, rate or extent of sarcinapterin biosynthetic process.